{
  "term_label": "Unknown cellular component",
  "gene": "UniProtKB:Q96T88",
  "gene_name": "E3 ubiquitin-protein ligase UHRF1",
  "gene_symbol": "UHRF1",
  "term_id": "UNKNOWN:0003"
}